gut granule assembly [GO:1902900] (biological process) Definition: The aggregation, arrangement and bonding together of a set of components to form a gut granule. References: PMID:17202409 Sources: GOC:TermGenie, GOC:kmv, GO_REF:0000079 Also known as: gut granule biogenesis, gut granule formation Relationships: is_a vesicle organization [GO:0016050]; is a type of organelle assembly [GO:0070925] Regulation: regulated by GO:1904755; negatively regulated by negative regulation of gut granule assembly [GO:1904756]; positively regulated by GO:1904757